{
  "term_label": "spermatid development",
  "gene_symbol": "SYCP3",
  "gene": "UniProtKB:Q8IZU3",
  "term_id": "GO:0007286",
  "gene_name": "Synaptonemal complex protein 3"
}